{
  "gene_name": "Alpha-actinin-1",
  "term_label": "cell junction",
  "term_id": "GO:0030054",
  "gene_symbol": "ACTN1",
  "gene": "UniProtKB:P12814"
}